{
  "term_id": "GO:0003700",
  "gene": "UniProtKB:Q8N1W2",
  "term_label": "DNA-binding transcription factor activity",
  "gene_name": "Zinc finger protein 710",
  "gene_symbol": "ZNF710"
}